{
  "gene_symbol": "CRIP1",
  "gene_name": "Cysteine-rich protein 1",
  "term_id": "GO:0008630",
  "term_label": "intrinsic apoptotic signaling pathway in response to DNA damage",
  "gene": "UniProtKB:P50238"
}